{
  "gene": "UniProtKB:Q8N4S9",
  "gene_symbol": "MARVELD2",
  "term_id": "GO:0070830",
  "gene_name": "MARVEL domain-containing protein 2",
  "term_label": "bicellular tight junction assembly"
}